{
  "term_id": "GO:0042278",
  "gene_symbol": "OARD1",
  "gene_name": "ADP-ribose glycohydrolase OARD1",
  "gene": "UniProtKB:Q9Y530",
  "term_label": "purine nucleoside metabolic process"
}